{
  "gene_name": "Protein CASC2, isoform 3",
  "gene": "UniProtKB:Q6XLA1",
  "gene_symbol": "CASC2",
  "term_label": "Unknown biological process",
  "term_id": "UNKNOWN:0002"
}